positive regulation of long-day photoperiodism, flowering [GO:0048578] (BP) Relationships: is a type of positive regulation of post-embryonic development [GO:0048582]; is_a positive regulation of response to stimulus [GO:0048584]; is a type of regulation of long-day photoperiodism, flowering [GO:0048586]; positively regulates long-day photoperiodism, flowering [GO:0048574] Sources: GOC:jid, GOC:pj, ISBN:0582015952, ISBN:0697037754, ISBN:0709408862 Also known as: up regulation of long-day photoperiodism, flowering, up-regulation of long-day photoperiodism, flowering, upregulation of long-day photoperiodism, flowering, activation of long-day photoperiodism, flowering, stimulation of long-day photoperiodism, flowering Definition: Any process that activates, maintains or increases long-day photoperiodism, where the response associated with the photoperiodism is flowering. Flowering is defined by the switch from the vegetative to the reproductive phase.